{
  "term_label": "plasma membrane",
  "term_id": "GO:0005886",
  "gene": "UniProtKB:Q6ZT62",
  "gene_name": "Bargin",
  "gene_symbol": "BARGIN"
}